{
  "gene_symbol": "TMEM62",
  "term_label": "Unknown biological process",
  "gene_name": "Transmembrane protein 62",
  "term_id": "UNKNOWN:0002",
  "gene": "UniProtKB:Q0P6H9"
}